{
  "term_id": "GO:0007129",
  "gene": "UniProtKB:Q8NA31",
  "gene_name": "Telomere repeats-binding bouquet formation protein 1",
  "term_label": "homologous chromosome pairing at meiosis",
  "gene_symbol": "TERB1"
}